regulation of thiamine biosynthetic process [GO:0070623] (biological process) Definition: Any process that modulates the frequency, rate or extent of the chemical reactions and pathways resulting in the formation of thiamine. Sources: GOC:mah Also known as: regulation of thiamin biosynthetic process, regulation of thiamine anabolism, regulation of thiamine biosynthesis, regulation of thiamine formation, regulation of thiamine synthesis Relationships: is a type of GO:0030656; is a type of regulation of sulfur metabolic process [GO:0042762]; is a type of regulation of alcohol biosynthetic process [GO:1902930]; regulates thiamine biosynthetic process [GO:0009228] Subtypes: negative regulation of thiamine biosynthetic process [GO:0070624], positive regulation of thiamine biosynthetic process [GO:0090180]